{
  "gene": "UniProtKB:A0A1W2PQ09",
  "gene_name": "TATA-box-binding protein-associated factor 11-like protein 11",
  "term_id": "GO:0005669",
  "gene_symbol": "TAF11L11",
  "term_label": "transcription factor TFIID complex"
}